nuclear membrane complex Bqt3-Bqt4 [GO:1990862] (cellular component) References: PMID:19948484 Relationships: is a type of membrane protein complex [GO:0098796]; is a type of nuclear protein-containing complex [GO:0140513]; is part of GO:0005637 Definition: A protein complex that resides in the inner nuclear membrane and anchors telomeres to the nuclear envelope. In fission yeast, it is composed of Bqt3 and Bqt4.